thorax and anterior abdomen determination [GO:0007356] (biological process) Definition: Specification of the central (trunk) regions of the embryo by the gap genes; exemplified in insects by the actions of the Kruppel gene product. Sources: ISBN:0879694238, http://fly.ebi.ac.uk/allied-data/lk/interactive-fly/aimain/1aahome.htm Relationships: is a type of anterior/posterior pattern specification [GO:0009952]; is part of zygotic determination of anterior/posterior axis, embryo [GO:0007354]